{
  "gene_symbol": "DYNLRB1",
  "term_label": "centrosome",
  "gene": "UniProtKB:Q9NP97",
  "term_id": "GO:0005813",
  "gene_name": "Dynein light chain roadblock-type 1"
}